(S,S)-butanediol dehydrogenase activity [GO:0047512] (molecular function) Sources: EC:1.1.1.76, RHEA:12184 Relationships: is a type of oxidoreductase activity, acting on the CH-OH group of donors, NAD or NADP as acceptor [GO:0016616] Definition: Catalysis of the reaction: (S,S)-butane-2,3-diol + NAD+ = acetoin + H+ + NADH. Also known as: (S,S)-butane-2,3-diol:NAD+ oxidoreductase activity, L(+)-2,3-butanediol dehydrogenase (L-acetoin forming), L-BDH, L-butanediol dehydrogenase activity